{
  "gene_symbol": "CALHM2",
  "term_id": "GO:0005886",
  "gene": "UniProtKB:Q9HA72",
  "term_label": "plasma membrane",
  "gene_name": "Calcium homeostasis modulator protein 2"
}